inter-Golgi cisterna vesicle-mediated transport [GO:0048219] (biological process) References: PMID:10219233 Sources: GOC:jid, GOC:mah, ISBN:0716731363 Also known as: inter-Golgi cisterna transport Relationships: is a type of intra-Golgi vesicle-mediated transport [GO:0006891] Definition: The directed movement of substances from one Golgi cisterna to another, mediated by small transport vesicles.